endonucleolytic cleavage to generate mature 5'-end of SSU-rRNA from (SSU-rRNA, 5.8S rRNA, LSU-rRNA) [GO:0000472] (biological process) Also known as: endonucleolytic cleavage at A1 References: PMID:10690410 Sources: GOC:curators Relationships: is a type of GO:0000479; is a type of GO:0000967; is part of maturation of SSU-rRNA from tricistronic rRNA transcript (SSU-rRNA, 5.8S rRNA, LSU-rRNA) [GO:0000462] Definition: Endonucleolytic cleavage between the 5'-External Transcribed Spacer (5'-ETS) and the 5' end of the SSU-rRNA of a tricistronic rRNA transcript that contains the Small Subunit (SSU) rRNA, the 5.8S rRNA, and the Large Subunit (LSU) rRNA in that order from 5' to 3' along the primary transcript, to produce the mature end of the SSU-rRNA.